nucleolus-like body [GO:1990934] (cellular component) Relationships: is a type of GO:0043232; is part of nuclear lumen [GO:0031981] Definition: A nuclear compartment containing significant amounts of non-nucleolar, spliceosomal components. It is commonly found in germinal vesicle (GV) stage oocytes, and is similar to both nucleoli and sphere organelles. References: PMID:26226217, PMID:9021878 Also known as: NLB, compact nucleolus